{
  "term_id": "GO:0016616",
  "gene": "UniProtKB:Q8IZV5",
  "term_label": "oxidoreductase activity, acting on the CH-OH group of donors, NAD or NADP as acceptor",
  "gene_name": "Retinol dehydrogenase 10",
  "gene_symbol": "RDH10"
}